{
  "gene_name": "Transmembrane protein 106C",
  "gene": "UniProtKB:Q9BVX2",
  "term_id": "UNKNOWN:0001",
  "term_label": "Unknown molecular function",
  "gene_symbol": "TMEM106C"
}